{
  "gene_symbol": "GATD3",
  "gene_name": "Glutamine amidotransferase-like class 1 domain-containing protein 3, mitochondrial",
  "term_id": "UNKNOWN:0001",
  "term_label": "Unknown molecular function",
  "gene": "UniProtKB:P0DPI2"
}